{
  "gene_symbol": "NEUROG3",
  "gene_name": "Neurogenin-3",
  "term_label": "DNA-binding transcription factor activity, RNA polymerase II-specific",
  "term_id": "GO:0000981",
  "gene": "UniProtKB:Q9Y4Z2"
}